{
  "term_id": "GO:0006346",
  "term_label": "DNA methylation-dependent constitutive heterochromatin formation",
  "gene": "UniProtKB:A0A1B0GVZ6",
  "gene_name": "Methyl-CpG-binding domain protein 3-like 2B",
  "gene_symbol": "MBD3L2B"
}